{
  "term_id": "GO:0005886",
  "term_label": "plasma membrane",
  "gene_symbol": "MS4A1",
  "gene_name": "B-lymphocyte antigen CD20",
  "gene": "UniProtKB:P11836"
}